{
  "gene": "UniProtKB:Q5T5B0",
  "term_id": "UNKNOWN:0002",
  "gene_name": "Late cornified envelope protein 3E",
  "term_label": "Unknown biological process",
  "gene_symbol": "LCE3E"
}